mesoderm structural organization [GO:0048338] (biological process) Also known as: mesoderm structural organisation Definition: The process that contributes to the act of creating the structural organization of the mesoderm. This process pertains to the physical shaping of a rudimentary structure. Relationships: is a type of anatomical structure arrangement [GO:0048532]; is part of mesoderm morphogenesis [GO:0048332] Subtypes: GO:0048331, GO:0048352, GO:0048381, intermediate mesoderm structural organization [GO:0048402] Sources: GOC:dgh